{
  "gene": "UniProtKB:A6NEN9",
  "gene_name": "Uncharacterized protein CXorf65",
  "gene_symbol": "CXorf65",
  "term_label": "Unknown cellular component",
  "term_id": "UNKNOWN:0003"
}